pinene metabolic process [GO:0033073] (biological process) Definition: The chemical reactions and pathways involving the monoterpenoid pinene; alpha-pinene is (1S,5S)-2,6,6-trimethylbicyclo[3.1.1]hept-2-ene, and beta-pinene is (1S,5S)-6,6-dimethyl-2-methylenebicyclo[3.1.1]heptane. Relationships: is a type of monoterpene metabolic process [GO:0043692] References: PMID:12623076 Sources: GOC:mah Subtypes: alpha-pinene metabolic process [GO:0018867], pinene catabolic process [GO:0033074] Also known as: pinene metabolism